type 3 metabotropic glutamate receptor binding [GO:0031800] (molecular function) Also known as: type 3 metabotropic glutamate receptor ligand Sources: GOC:mah, GOC:nln Definition: Binding to a type 3 metabotropic glutamate receptor. Relationships: is a type of G protein-coupled glutamate receptor binding [GO:0035256]